response to mannose [GO:1905582] (biological process) Subtypes: cellular response to mannose [GO:1905583] References: PMID:16699509 Sources: GOC:TermGenie, GO_REF:0000071 Relationships: is a type of GO:0009746 Definition: Any process that results in a change in state or activity of a cell or an organism (in terms of movement, secretion, enzyme production, gene expression, etc.) as a result of a mannose stimulus.